{
  "gene_name": "Synaptogyrin-2",
  "term_label": "Unknown biological process",
  "gene_symbol": "SYNGR2",
  "gene": "UniProtKB:O43760",
  "term_id": "UNKNOWN:0002"
}